{
  "term_id": "GO:0005912",
  "gene_name": "Cadherin-10",
  "gene": "UniProtKB:Q9Y6N8",
  "term_label": "adherens junction",
  "gene_symbol": "CDH10"
}